cell junction organization [GO:0034330] (biological process) Sources: GOC:dph, GOC:jl, GOC:mah Subtypes: cell junction assembly [GO:0034329], cell junction maintenance [GO:0034331], GO:0045216, GO:0050808, flagellum attachment zone organization [GO:0110140], cell-substrate junction organization [GO:0150115], cell junction disassembly [GO:0150146] Definition: A process that is carried out at the cellular level which results in the assembly, arrangement of constituent parts, or disassembly of a cell junction. A cell junction is a specialized region of connection between two cells or between a cell and the extracellular matrix. Also known as: cell junction assembly and maintenance, cell junction organisation, cell junction biogenesis Relationships: is a type of cellular component organization [GO:0016043]